glutathione thiolesterase activity [GO:0047951] (molecular function) Definition: Catalysis of the reaction: S-acylglutathione + H2O = a carboxylate + glutathione + H+. Relationships: is a type of thiolester hydrolase activity [GO:0016790] Also known as: glutathione thioesterase activity, S-acylglutathione hydrolase activity, citryl-glutathione thioesterhydrolase activity Sources: EC:3.1.2.7, RHEA:22708